{
  "term_label": "Unknown molecular function",
  "gene": "UniProtKB:Q01628",
  "term_id": "UNKNOWN:0001",
  "gene_symbol": "IFITM3",
  "gene_name": "Interferon-induced transmembrane protein 3"
}